{
  "gene": "UniProtKB:Q5VU92",
  "term_label": "Unknown biological process",
  "gene_name": "DDB1- and CUL4-associated factor 12-like protein 1",
  "term_id": "UNKNOWN:0002",
  "gene_symbol": "DCAF12L1"
}